{
  "gene": "UniProtKB:Q9H000",
  "term_label": "protein ubiquitination",
  "gene_symbol": "MKRN2",
  "term_id": "GO:0016567",
  "gene_name": "E3 ubiquitin-protein ligase makorin-2"
}